{
  "term_id": "GO:0006357",
  "gene_name": "Zinc finger protein 835",
  "gene_symbol": "ZNF835",
  "term_label": "regulation of transcription by RNA polymerase II",
  "gene": "UniProtKB:Q9Y2P0"
}